cholestenol delta-isomerase activity [GO:0047750] (molecular function) Definition: Catalysis of the reaction: 5-alpha-cholest-7-en-3-beta-ol = 5-alpha-cholest-8-en-3-beta-ol. Sources: RHEA:15281 Also known as: cholestenol D-isomerase activity, delta7-cholestenol delta7-delta8-isomerase activity Relationships: is a type of intramolecular oxidoreductase activity, transposing C=C bonds [GO:0016863]